methylthioribulose 1-phosphate dehydratase activity [GO:0046570] (molecular function) Definition: Catalysis of the reaction: S-methyl-5-thio-D-ribulose 1-phosphate = 5-(methylthio)-2,3-dioxopentyl phosphate + H2O. Sources: EC:4.2.1.109, RHEA:15549 Also known as: 5-methylthioribulose-1-phosphate 4-dehydratase activity, S-methyl-5-thio-D-ribulose-1-phosphate hydro-lyase activity, S-methyl-5-thio-D-ribulose-1-phosphate hydro-lyase[5-(methylthio)-2,3-dioxopentyl-phosphate-forming], methylthioribulose-1-phosphate dehydratase activity, 1-PMT-ribulose dehydratase activity, S-methyl-5-thio-D-ribulose-1-phosphate hydro-lyase [5-(methylthio)-2,3-dioxopentyl-phosphate-forming] Relationships: is_a hydro-lyase activity [GO:0016836]